{
  "gene_name": "Zinc finger protein 680",
  "term_id": "GO:0000981",
  "term_label": "DNA-binding transcription factor activity, RNA polymerase II-specific",
  "gene_symbol": "ZNF680",
  "gene": "UniProtKB:Q8NEM1"
}